{
  "term_id": "UNKNOWN:0002",
  "gene": "UniProtKB:C0HM01",
  "gene_name": "Putative RNA-binding regulatory peptide",
  "gene_symbol": "SEPTIN14P20",
  "term_label": "Unknown biological process"
}